protein polyamination [GO:0018184] (biological process) Relationships: is a type of protein modification process [GO:0036211] Sources: GOC:ai Definition: The modification of a protein amino acid by polyamination. Also known as: protein amino acid polyamination